{
  "term_id": "GO:0004903",
  "gene": "UniProtKB:P10912",
  "gene_name": "Growth hormone receptor",
  "term_label": "growth hormone receptor activity",
  "gene_symbol": "GHR"
}